gamma-glutamyl carboxylase activity [GO:0008488] (molecular function) References: PMID:18374194 Definition: Catalysis of the reaction: peptidyl-glutamate + reduced vitamin K + CO2 + O2 = peptidyl-gamma-carboxyglutamate + vitamin K epoxide. Relationships: is a type of carboxy-lyase activity [GO:0016831]